{
  "term_label": "Golgi membrane",
  "gene": "UniProtKB:Q9Y5U9",
  "gene_symbol": "IER3IP1",
  "term_id": "GO:0000139",
  "gene_name": "Immediate early response 3-interacting protein 1"
}